{
  "term_label": "arachidonate-CoA ligase activity",
  "gene_symbol": "ACSL5",
  "term_id": "GO:0047676",
  "gene_name": "Long-chain-fatty-acid--CoA ligase 5",
  "gene": "UniProtKB:Q9ULC5"
}